{
  "term_id": "UNKNOWN:0003",
  "gene_symbol": "WDR86",
  "gene": "UniProtKB:Q86TI4",
  "term_label": "Unknown cellular component",
  "gene_name": "WD repeat-containing protein 86"
}